{
  "gene_symbol": "SPAG11A",
  "term_id": "UNKNOWN:0003",
  "gene_name": "Sperm-associated antigen 11A",
  "gene": "UniProtKB:Q6PDA7",
  "term_label": "Unknown cellular component"
}